{
  "term_label": "spliceosomal tri-snRNP complex",
  "term_id": "GO:0097526",
  "gene_symbol": "SNRPGP15",
  "gene": "UniProtKB:A8MWD9",
  "gene_name": "Putative small nuclear ribonucleoprotein G-like protein 15"
}